{
  "gene": "UniProtKB:Q9C0K1",
  "term_label": "plasma membrane",
  "gene_symbol": "SLC39A8",
  "term_id": "GO:0005886",
  "gene_name": "Metal cation symporter ZIP8"
}